{
  "gene": "UniProtKB:P02708",
  "term_label": "monoatomic ion transmembrane transport",
  "gene_symbol": "CHRNA1",
  "term_id": "GO:0034220",
  "gene_name": "Acetylcholine receptor subunit alpha"
}